{
  "term_label": "proteoglycan binding",
  "term_id": "GO:0043394",
  "gene": "UniProtKB:P02751",
  "gene_symbol": "FN1",
  "gene_name": "Fibronectin"
}